photoreceptor cell fate determination [GO:0043703] (biological process) Definition: The process in which a cell becomes capable of differentiating autonomously into a photoreceptor cell regardless of its environment; upon determination, the cell fate cannot be reversed. Relationships: is a type of neuron fate determination [GO:0048664]; is part of photoreceptor cell fate commitment [GO:0046552] Subtypes: retinal cone cell fate determination [GO:0042671] Sources: GOC:mtg_sensu